{
  "term_label": "oxidoreductase activity",
  "gene_name": "Iodotyrosine deiodinase 1",
  "gene": "UniProtKB:Q6PHW0",
  "term_id": "GO:0016491",
  "gene_symbol": "IYD"
}